{
  "term_label": "cholesterol homeostasis",
  "gene_name": "Oxysterols receptor LXR-beta",
  "gene": "UniProtKB:P55055",
  "gene_symbol": "NR1H2",
  "term_id": "GO:0042632"
}